5'-tyrosyl-DNA phosphodiesterase activity [GO:0070260] (molecular function) Relationships: is a type of tyrosyl-DNA phosphodiesterase activity [GO:0070259] Definition: Catalysis of the hydrolysis of 5'-phosphotyrosyl groups formed as covalent intermediates (in DNA backbone breakage) between DNA topoisomerase II and DNA. References: PMID:16751265 Note: See also the molecular function term 'DNA topoisomerase type I activity ; GO:0003917'.